peptidyl-lysine oxidation [GO:0018057] (biological process) Relationships: is a type of protein oxidation [GO:0018158]; is_a GO:0018205 Sources: ISBN:0198547684, RESID:AA0121 Definition: The oxidation of the terminal amino-methylene groups of peptidyl-L-lysine or peptidyl-5-hydroxy-L-lysine to aldehyde groups to form allysine or hydroxyallysine residues, respectively; these are intermediates in the formation of covalent cross-links between adjacent polypeptide chains in proteins such as collagens.